camera-type eye photoreceptor cell development [GO:0062139] (biological process) Definition: The process whose specific outcome is the progression of a light-responsive receptor in a camera-type eye over time, from its formation to the mature structure. Relationships: is a type of eye photoreceptor cell development [GO:0042462]; is part of camera-type eye development [GO:0043010] References: PMID:20648062, PMID:30237290